methanopterin-containing compound biosynthetic process [GO:2001116] (biological process) Subtypes: GO:1900868, GO:2001118 Relationships: is_a phosphate-containing compound metabolic process [GO:0006796]; is a type of pteridine-containing compound biosynthetic process [GO:0042559]; is_a organophosphate biosynthetic process [GO:0090407] Definition: The chemical reactions and pathways resulting in the formation of a methanopterin. Also known as: methanopterin biosynthesis Sources: GOC:mengo_curators